{
  "gene_symbol": "CHRNA2",
  "gene": "UniProtKB:Q15822",
  "gene_name": "Neuronal acetylcholine receptor subunit alpha-2",
  "term_label": "synapse",
  "term_id": "GO:0045202"
}